positive regulation of aldosterone secretion [GO:2000860] (biological process) Definition: Any process that activates or increases the frequency, rate or extent of aldosterone secretion. Relationships: is a type of positive regulation of mineralocorticoid secretion [GO:2000857]; is a type of regulation of aldosterone secretion [GO:2000858]; positively regulates aldosterone secretion [GO:0035932] Sources: GOC:sl